{
  "term_id": "UNKNOWN:0002",
  "term_label": "Unknown biological process",
  "gene": "UniProtKB:Q96CN5",
  "gene_name": "Leucine-rich repeat-containing protein 45",
  "gene_symbol": "LRRC45"
}